{
  "term_id": "GO:0000977",
  "gene_name": "Autoimmune regulator",
  "term_label": "RNA polymerase II transcription regulatory region sequence-specific DNA binding",
  "gene_symbol": "AIRE",
  "gene": "UniProtKB:O43918"
}